{
  "gene_symbol": "EFCAB8",
  "gene": "UniProtKB:A8MWE9",
  "term_id": "UNKNOWN:0002",
  "gene_name": "EF-hand calcium-binding domain-containing protein 8",
  "term_label": "Unknown biological process"
}